{
  "gene_symbol": "AP4S1",
  "term_id": "GO:0016192",
  "gene": "UniProtKB:Q9Y587",
  "gene_name": "AP-4 complex subunit sigma-1",
  "term_label": "vesicle-mediated transport"
}